2-aminoethylphosphonate binding [GO:0033226] (molecular function) Sources: GOC:mlg Also known as: 2-phosphonoethylamine binding, ciliatine binding Relationships: is a type of small molecule binding [GO:0036094] Definition: Binding to 2-aminoethylphosphonate.